{
  "gene_name": "Apoptotic protease-activating factor 1",
  "gene_symbol": "APAF1",
  "gene": "UniProtKB:O14727",
  "term_label": "Unknown cellular component",
  "term_id": "UNKNOWN:0003"
}